{
  "gene": "UniProtKB:O95453",
  "gene_symbol": "PARN",
  "term_id": "GO:0000289",
  "gene_name": "Poly(A)-specific ribonuclease PARN",
  "term_label": "nuclear-transcribed mRNA poly(A) tail shortening"
}